sensory perception of electrical stimulus [GO:0050952] (biological process) Relationships: is a type of sensory perception [GO:0007600] Sources: GOC:ai Subtypes: electroception [GO:0050956], magnetoreception by sensory perception of electrical stimulus [GO:0050978] Definition: The series of events required for an organism to receive a sensory electrical stimulus, convert it to a molecular signal, and recognize and characterize the signal. This is a neurological process.